{
  "term_id": "GO:0030687",
  "gene_name": "60S ribosome subunit biogenesis protein NIP7 homolog",
  "gene": "UniProtKB:Q9Y221",
  "term_label": "preribosome, large subunit precursor",
  "gene_symbol": "NIP7"
}